cytoplasmic side of dendritic spine plasma membrane [GO:1990780] (cellular component) Definition: The leaflet of the plasma membrane that faces the cytoplasm and any proteins embedded or anchored in it or attached to its surface surrounding a dendritic spine. Relationships: is a type of cytoplasmic side of plasma membrane [GO:0009898]; BFO_0000050 dendritic spine membrane [GO:0032591] References: PMID:9275233